gland development [GO:0048732] (biological process) Relationships: is a type of animal organ development [GO:0048513] Definition: The process whose specific outcome is the progression of a gland over time, from its formation to the mature structure. A gland is an organ specialised for secretion. Subtypes: GO:0001889, salivary gland development [GO:0007431], pineal gland development [GO:0021982], pituitary gland development [GO:0021983], GO:0021985, GO:0030325, prostate gland development [GO:0030850], thyroid gland development [GO:0030878], mammary gland development [GO:0030879], GO:0031017, lacrimal gland development [GO:0032808], ring gland development [GO:0035271], thymus development [GO:0048538], lymph gland development [GO:0048542], sebaceous gland development [GO:0048733], hatching gland development [GO:0048785], parathyroid gland development [GO:0060017], sweat gland development [GO:0060792], seminal vesicle development [GO:0061107], trachea gland development [GO:0061153], GO:0070384, cement gland development [GO:0071570], uterine gland development [GO:1903709], cloacal gland development [GO:1904484] Sources: GOC:jid